viomycin kinase activity [GO:0050394] (molecular function) Definition: Catalysis of the reaction: ATP + viomycin = ADP + O-phosphoviomycin. Sources: EC:2.7.1.103, MetaCyc:VIOMYCIN-KINASE-RXN Also known as: ATP:viomycin O-phosphotransferase activity, capreomycin phosphotransferase activity, viomycin phosphotransferase activity Relationships: is a type of GO:0016301; is a type of phosphotransferase activity, alcohol group as acceptor [GO:0016773]